{
  "gene_symbol": "RHOBTB1",
  "term_label": "actin filament organization",
  "gene": "UniProtKB:O94844",
  "gene_name": "Rho-related BTB domain-containing protein 1",
  "term_id": "GO:0007015"
}